{
  "term_label": "cellular response to oxidative stress",
  "term_id": "GO:0034599",
  "gene": "UniProtKB:O75715",
  "gene_name": "Epididymal secretory glutathione peroxidase",
  "gene_symbol": "GPX5"
}